{
  "gene_symbol": "RAP2C",
  "term_id": "GO:0032486",
  "gene_name": "Ras-related protein Rap-2c",
  "gene": "UniProtKB:Q9Y3L5",
  "term_label": "Rap protein signal transduction"
}